{
  "gene_symbol": "GRIP2",
  "term_id": "UNKNOWN:0003",
  "term_label": "Unknown cellular component",
  "gene": "UniProtKB:Q9C0E4",
  "gene_name": "Glutamate receptor-interacting protein 2"
}